3-deoxyglucosone dehydrogenase activity [GO:0106373] (molecular function) References: PMID:17175089 Sources: RHEA:67244 Definition: Catalysis of the reaction: 3-deoxyglucosone + H2O + NAD+ = 2-dehydro-3-deoxy-D-gluconate + 2 H+ + NADH. Relationships: is a type of aldehyde dehydrogenase (NAD+) activity [GO:0004029]